{
  "gene_symbol": "ARRDC2",
  "gene": "UniProtKB:Q8TBH0",
  "gene_name": "Arrestin domain-containing protein 2",
  "term_id": "GO:0005886",
  "term_label": "plasma membrane"
}